{
  "gene": "UniProtKB:Q9UHT4",
  "gene_symbol": "PRO1854",
  "term_id": "UNKNOWN:0003",
  "gene_name": "Putative uncharacterized protein PRO1854",
  "term_label": "Unknown cellular component"
}